{
  "term_label": "Unknown molecular function",
  "term_id": "UNKNOWN:0001",
  "gene": "UniProtKB:Q7RTP0",
  "gene_name": "Magnesium transporter NIPA1",
  "gene_symbol": "NIPA1"
}